{
  "gene_name": "Major facilitator superfamily domain-containing protein 6-like",
  "gene": "UniProtKB:Q8IWD5",
  "term_label": "Unknown molecular function",
  "term_id": "UNKNOWN:0001",
  "gene_symbol": "MFSD6L"
}